early neuron fate commitment in forebrain [GO:0021901] (biological process) References: PMID:16226447 Sources: GOC:cls, GOC:dgh, GOC:dph, GOC:jid, GO_REF:0000021 Relationships: is a type of commitment of multipotent stem cells to neuronal lineage in forebrain [GO:0021898]; is part of GO:0021862 Definition: The commitment of neuroepithelial cell to become a neuron that will reside in the forebrain.